{
  "term_label": "GTPase activity",
  "gene": "UniProtKB:Q15907",
  "gene_name": "Ras-related protein Rab-11B",
  "gene_symbol": "RAB11B",
  "term_id": "GO:0003924"
}